{
  "gene": "UniProtKB:O94983",
  "term_label": "double-stranded DNA binding",
  "term_id": "GO:0003690",
  "gene_name": "Calmodulin-binding transcription activator 2",
  "gene_symbol": "CAMTA2"
}